{
  "gene_symbol": "IFITM1",
  "gene_name": "Interferon-induced transmembrane protein 1",
  "gene": "UniProtKB:P13164",
  "term_label": "response to interferon-alpha",
  "term_id": "GO:0035455"
}